{
  "term_label": "integrin binding",
  "gene_symbol": "JAM3",
  "term_id": "GO:0005178",
  "gene": "UniProtKB:Q9BX67",
  "gene_name": "Junctional adhesion molecule C"
}